{
  "term_label": "T cell receptor signaling pathway",
  "gene_symbol": "FYB1",
  "gene_name": "FYN-binding protein 1",
  "term_id": "GO:0050852",
  "gene": "UniProtKB:O15117"
}